{
  "gene": "UniProtKB:Q15768",
  "gene_name": "Ephrin-B3",
  "term_id": "GO:0005886",
  "gene_symbol": "EFNB3",
  "term_label": "plasma membrane"
}